polysaccharide immune receptor activity [GO:0001873] (molecular function) Relationships: is_a pattern recognition receptor activity [GO:0038187]; has part GO:0030247 Subtypes: GO:0001874 References: PMID:14707091 Also known as: polysaccharide receptor activity Definition: Combining with a polysaccharide and transmitting the signal to initiate an innate immune response. A polysaccharide is a polymer of many (typically more than 10) monosaccharide residues linked glycosidically.